positive regulation of 5-methylcytosine DNA demethylation, direct 5-methylcytosine excision pathway [GO:0141170] (biological process) Definition: Any process that activates or increases the frequency, rate or extent of positive regulation of 5-methylcytosine DNA demethylation, direct 5-methylcytosine excision pathway. References: PMID:36478523 Relationships: is a type of GO:0051054; positively regulates GO:0141169